{
  "term_id": "GO:0006511",
  "gene": "UniProtKB:Q9ULT6",
  "gene_symbol": "ZNRF3",
  "gene_name": "E3 ubiquitin-protein ligase ZNRF3",
  "term_label": "ubiquitin-dependent protein catabolic process"
}